regulation of phagosome maturation [GO:1905162] (BP) Relationships: is a type of regulation of organelle organization [GO:0033043]; regulates GO:0090382 References: PMID:16908865, PMID:23303671 Sources: GOC:PARL, GOC:TermGenie, GOC:bf, GO_REF:0000058 Definition: Any process that modulates the frequency, rate or extent of phagosome maturation. Subtypes: negative regulation of phagosome maturation [GO:1905163], GO:1905164